D-glucarate catabolic process [GO:0042838] (biological process) Also known as: D-glucarate breakdown, D-glucarate catabolism, D-glucarate degradation, saccharate catabolic process, saccharate catabolism Relationships: is a type of GO:0016052; is a type of GO:0019394; is a type of D-glucarate metabolic process [GO:0042836] Sources: GOC:jsg, GOC:mah, ISBN:0198506732 Definition: The chemical reactions and pathways resulting in the breakdown of D-glucarate, the D-enantiomer of glucarate.